{
  "term_label": "vesicle-mediated transport",
  "gene_symbol": "AP4B1",
  "gene": "UniProtKB:Q9Y6B7",
  "gene_name": "AP-4 complex subunit beta-1",
  "term_id": "GO:0016192"
}